response to zinc ion starvation [GO:0120127] (biological process) Definition: Any process that results in a change in state or activity of a cell or an organism (in terms of movement, secretion, enzyme production, gene expression, etc.) as a result of a starvation stimulus, deprivation of zinc ion. Relationships: is a type of response to metal ion starvation [GO:0180055] References: PMID:24024381 Sources: GOC:sl Subtypes: cellular response to zinc ion starvation [GO:0034224]